ERBB4:ERBB2 complex [GO:0038144] (cellular component) Definition: A heterodimeric complex between the tyrosine kinase receptor ERBB2 and a ligand-activated receptor ERBB4. ERBB2, which does not bind any known ligand, is activated through formation of a heterodimer with another ligand-activated ERBB family member such as ERBB4. References: PMID:16460914, PMID:16978839 Sources: GOC:signaling Also known as: ERBB4:ERBB2 heterodimer, NRGs/EGFLs:ERBB4:ERBB2 Relationships: is a type of plasma membrane signaling receptor complex [GO:0098802]